{
  "gene_symbol": "SPDL1",
  "gene_name": "Protein Spindly",
  "term_label": "mitotic metaphase chromosome alignment",
  "term_id": "GO:0007080",
  "gene": "UniProtKB:Q96EA4"
}